regulation of embryonic skeletal joint development [GO:1902762] (biological process) Definition: Any process that modulates the frequency, rate or extent of embryonic skeletal joint development. References: PMID:16575901 Sources: GOC:TermGenie, GOC:mr, GO_REF:0000058 Subtypes: GO:1902763, positive regulation of embryonic skeletal joint development [GO:1902764] Relationships: is a type of regulation of developmental process [GO:0050793]; regulates embryonic skeletal joint development [GO:0072498]